morphogenesis of follicular epithelium [GO:0016333] (biological process) Definition: The process in which the anatomical structures of a follicular epithelium are generated and organized. Sources: GOC:jl Relationships: is a type of morphogenesis of an epithelium [GO:0002009]